{
  "term_label": "antigen binding",
  "gene": "UniProtKB:P01861",
  "gene_name": "Immunoglobulin heavy constant gamma 4",
  "gene_symbol": "IGHG4",
  "term_id": "GO:0003823"
}